{
  "gene": "UniProtKB:Q96MU7",
  "gene_symbol": "YTHDC1",
  "term_label": "mRNA splicing, via spliceosome",
  "term_id": "GO:0000398",
  "gene_name": "YTH domain-containing protein 1"
}